{
  "gene_symbol": "CEACAM16",
  "term_id": "UNKNOWN:0003",
  "gene_name": "Carcinoembryonic antigen-related cell adhesion molecule 16",
  "term_label": "Unknown cellular component",
  "gene": "UniProtKB:Q2WEN9"
}